{
  "term_id": "GO:0005736",
  "gene_symbol": "POLR2H",
  "term_label": "RNA polymerase I complex",
  "gene": "UniProtKB:P52434",
  "gene_name": "DNA-directed RNA polymerases I, II, and III subunit RPABC3"
}